{
  "gene_symbol": "THAP9",
  "gene": "UniProtKB:Q9H5L6",
  "gene_name": "DNA transposase THAP9",
  "term_label": "Unknown cellular component",
  "term_id": "UNKNOWN:0003"
}